{
  "gene": "UniProtKB:Q13501",
  "gene_symbol": "SQSTM1",
  "term_label": "endosome organization",
  "term_id": "GO:0007032",
  "gene_name": "Sequestosome-1"
}